{
  "gene_name": "Appetite-regulating hormone",
  "gene_symbol": "GHRL",
  "term_id": "GO:0005615",
  "gene": "UniProtKB:Q9UBU3",
  "term_label": "extracellular space"
}